{
  "term_label": "Unknown biological process",
  "gene_name": "Olfactory receptor 6V1",
  "gene": "UniProtKB:Q8N148",
  "gene_symbol": "OR6V1",
  "term_id": "UNKNOWN:0002"
}